positive regulation of potassium ion export across plasma membrane [GO:1903766] (biological process) Relationships: is a type of GO:1901381; is a type of regulation of potassium ion export across plasma membrane [GO:1903764]; positively regulates potassium ion export across plasma membrane [GO:0097623] Also known as: positive regulation of potassium export, positive regulation of potassium ion export, up regulation of potassium export, up regulation of potassium ion export, up-regulation of potassium export, up-regulation of potassium ion export, upregulation of potassium export, upregulation of potassium ion export, up regulation of potassium ion export across plasma membrane, up-regulation of potassium ion export across plasma membrane, upregulation of potassium ion export across plasma membrane, activation of potassium export, activation of potassium ion export, activation of potassium ion export across plasma membrane References: PMID:19646991 Sources: GOC:BHF, GOC:TermGenie, GOC:mtg_cardiac_conduct_nov11, GOC:rl, GO_REF:0000058 Definition: Any process that activates or increases the frequency, rate or extent of potassium ion export across the plasma membrane.